regulation of multicellular organismal process [GO:0051239] (biological process) Definition: Any process that modulates the frequency, rate or extent of a multicellular organismal process, the processes pertinent to the function of a multicellular organism above the cellular level; includes the integrated processes of tissues and organs. Subtypes: GO:0001817, regulation of epithelial cell migration [GO:0010632], regulation of very-low-density lipoprotein particle remodeling [GO:0010901], regulation of lipoprotein particle clearance [GO:0010984], GO:0014807, regulation of ossification [GO:0030278], regulation of heat generation [GO:0031650], GO:0031654, GO:0032899, regulation of tissue remodeling [GO:0034103], regulation of plasma lipoprotein oxidation [GO:0034444], regulation of hemocyte proliferation [GO:0035206], GO:0035490, GO:0040014, regulation of hair cycle [GO:0042634], GO:0043012, regulation of respiratory gaseous exchange [GO:0043576], regulation of system process [GO:0044057], GO:0045610, regulation of spermatid nuclear differentiation [GO:0045700], regulation of salivary gland boundary specification [GO:0045704], GO:0046620, GO:0048819, GO:0050795, regulation of coagulation [GO:0050818], regulation of cell activation [GO:0050865], positive regulation of multicellular organismal process [GO:0051240], negative regulation of multicellular organismal process [GO:0051241], GO:0060264, GO:0060278, regulation of penile erection [GO:0060405], GO:0060688, GO:0070255, regulation of pollen tube growth [GO:0080092], GO:0090107, regulation of radial pattern formation [GO:0090213], GO:0090318, GO:0090381, GO:0110107, regulation of cold-induced thermogenesis [GO:0120161], regulation of trichome patterning [GO:1900032], regulation of amyloid-beta clearance [GO:1900221], GO:1902490, regulation of embryonic pattern specification [GO:1902875], GO:1903186, regulation of fear response [GO:1903365], regulation of histamine secretion by mast cell [GO:1903593], regulation of epithelial cell-cell adhesion involved in epithelium migration [GO:1903681], GO:1904298, regulation of maternal process involved in parturition [GO:1904301], regulation of male germ-line stem cell asymmetric division [GO:1904838], regulation of oogenesis [GO:1905879], regulation of germ cell proliferation [GO:1905936], GO:2000011, regulation of determination of dorsal identity [GO:2000015], GO:2000026, GO:2000036, GO:2000037 Relationships: is a type of GO:0050789; regulates multicellular organismal process [GO:0032501] Sources: GOC:ai, GOC:dph, GOC:tb